1-deoxy-D-xylulose-5-phosphate reductoisomerase activity [GO:0030604] (molecular function) Definition: Catalysis of the reaction: 2-C-methyl-D-erythritol 4-phosphate + NADP+ = 1-deoxy-D-xylulose 5-phosphate + H+ + NADPH. Sources: EC:1.1.1.267, RHEA:13717 Relationships: is a type of GO:0016616 Also known as: DOXP reductoisomerase activity, 1-deoxy-D-xylulose-5-phosphate isomeroreductase activity, 1-deoxyxylulose-5-phosphate reductoisomerase activity, 2-C-methyl-D-erythritol-4-phosphate:NADP+ oxidoreductase (isomerizing), 2C-methyl-D-erythritol-4-phosphate (MEP) synthase activity, DXP-reductoisomerase activity